{
  "term_id": "GO:0005634",
  "gene_name": "BTB_POZ domain-containing protein 18",
  "term_label": "nucleus",
  "gene_symbol": "BTBD18",
  "gene": "UniProtKB:B2RXH4"
}